{
  "term_label": "plasma membrane",
  "term_id": "GO:0005886",
  "gene_symbol": "SLC19A3",
  "gene": "UniProtKB:Q9BZV2",
  "gene_name": "Thiamine transporter 2"
}